membrane biogenesis [GO:0044091] (biological process) Subtypes: GO:0016557, rhabdomere membrane biogenesis [GO:0045313], nuclear membrane biogenesis [GO:0101025], endoplasmic reticulum membrane biogenesis [GO:0160031] Sources: GOC:jl Relationships: is a type of cellular component biogenesis [GO:0044085] Definition: A cellular process that results in the biosynthesis of constituent macromolecules, assembly, and arrangement of constituent parts of a membrane.